ribosome hibernation [GO:0141014] (biological process) References: PMID:28468753, PMID:30177741, PMID:36653451 Definition: A cellular process that results in the silencing of ribosomes in quiescent cells. Quiescence takes place when cells encounter unfavorable conditions and cease to grow in bacteria and yeast. It also takes place in some specialized cells in higher eukaryotes, such as eggs. Ribosomes in a hibernation state are kept silent via association with proteins with inhibitory and protective functions. Relationships: is a type of GO:0017148